{
  "gene": "UniProtKB:A0A669KB60",
  "term_id": "UNKNOWN:0002",
  "term_label": "Unknown biological process",
  "gene_symbol": "A0A669KB60",
  "gene_name": "Uncharacterized protein"
}